purine ribonucleoside biosynthetic process [GO:0046129] (BP) Relationships: is_a purine nucleoside biosynthetic process [GO:0042451]; is a type of GO:0042455; is a type of GO:0046128 Definition: The chemical reactions and pathways resulting in the formation of any purine ribonucleoside, a nucleoside in which purine base is linked to a ribose (beta-D-ribofuranose) molecule. Subtypes: purine ribonucleoside salvage [GO:0006166], puromycin biosynthetic process [GO:0043638], adenosine biosynthetic process [GO:0046086], inosine biosynthetic process [GO:0046103], guanosine-containing compound biosynthetic process [GO:1901070], xanthosine biosynthetic process [GO:1903229] Sources: GOC:ai Also known as: purine ribonucleoside anabolism, purine ribonucleoside biosynthesis, purine ribonucleoside formation, purine ribonucleoside synthesis